corticotropin-releasing hormone receptor binding [GO:0051429] (molecular function) Also known as: CRF receptor binding, CRH receptor binding, CRHR binding, corticotropin releasing factor receptor binding, corticotropin-releasing factor receptor binding, corticotropin releasing factor receptor ligand Subtypes: corticotropin-releasing hormone receptor 1 binding [GO:0051430], corticotropin-releasing hormone receptor 2 binding [GO:0051431] Relationships: is a type of peptide hormone receptor binding [GO:0051428]; is a type of neuropeptide receptor binding [GO:0071855] Sources: GOC:ai Definition: Binding to a receptor for corticotropin-releasing hormone (CRH), a polypeptide hormone involved in the stress response. It is released by the hypothalamus and stimulates the release of corticotropin by the anterior pituitary gland.